{
  "gene_symbol": "DCTN4",
  "term_id": "UNKNOWN:0002",
  "gene": "UniProtKB:Q9UJW0",
  "gene_name": "Dynactin subunit 4",
  "term_label": "Unknown biological process"
}